{
  "term_id": "UNKNOWN:0001",
  "term_label": "Unknown molecular function",
  "gene_symbol": "PROCR",
  "gene_name": "Endothelial protein C receptor",
  "gene": "UniProtKB:Q9UNN8"
}